{
  "gene_name": "Beta-glucuronidase",
  "term_label": "extracellular space",
  "term_id": "GO:0005615",
  "gene_symbol": "GUSB",
  "gene": "UniProtKB:P08236"
}